{
  "term_id": "GO:0006887",
  "gene_symbol": "EXOC7",
  "term_label": "exocytosis",
  "gene": "UniProtKB:Q9UPT5",
  "gene_name": "Exocyst complex component 7"
}